{
  "term_label": "nucleus",
  "gene": "UniProtKB:P05161",
  "gene_symbol": "ISG15",
  "term_id": "GO:0005634",
  "gene_name": "Ubiquitin-like protein ISG15"
}